{
  "gene_name": "Zinc finger protein 717",
  "term_label": "negative regulation of transcription by RNA polymerase II",
  "gene": "UniProtKB:Q9BY31",
  "gene_symbol": "ZNF717",
  "term_id": "GO:0000122"
}